{
  "gene": "UniProtKB:O95394",
  "term_id": "GO:0006048",
  "gene_name": "Phosphoacetylglucosamine mutase",
  "term_label": "UDP-N-acetylglucosamine biosynthetic process",
  "gene_symbol": "PGM3"
}